{
  "term_label": "Unknown biological process",
  "gene_name": "Transcription elongation factor A protein-like 2",
  "gene": "UniProtKB:Q9H3H9",
  "gene_symbol": "TCEAL2",
  "term_id": "UNKNOWN:0002"
}